{
  "term_id": "GO:0007267",
  "gene_name": "Pannexin-1",
  "gene_symbol": "PANX1",
  "term_label": "cell-cell signaling",
  "gene": "UniProtKB:Q96RD7"
}